leak channel activity [GO:0022840] (molecular function) Relationships: is a type of narrow pore channel activity [GO:0022842] Subtypes: GO:0022841 Definition: Enables the transport of a solute across a membrane via a narrow pore channel that is open even in an unstimulated or 'resting' state. Sources: GOC:mtg_transport, ISBN:0815340729